{
  "term_id": "GO:0046579",
  "gene_name": "Serine_threonine-protein kinase 19",
  "term_label": "positive regulation of Ras protein signal transduction",
  "gene_symbol": "STK19",
  "gene": "UniProtKB:P49842"
}